heteromeric SMAD protein complex [GO:0071144] (cellular component) Definition: A protein complex composed of SMAD family proteins, a transcription factor complex which binds to the promoters of target genes and recruits co-activators and histone acetyltransferases, facilitating transcription. Phosphorylation of the non-SMAD4 subunit(s) enables binding of SMAD4 to form heteromeric complexes that enter the nucleus to initiate gene transcription. DNA-binding specificity is conferred by other transcription factors binding to SMAD complexes. Interactions with coactivators or corepressors modulate their transcriptional activity. Can be heterotrimeric or heterodimeric. References: PMID:11779505, PMID:15350224, PMID:16322555, PMID:9389648, PMID:9670020 Sources: GOC:bhm, GOC:mah Relationships: is a type of SMAD protein complex [GO:0071141]; is a type of RNA polymerase II transcription regulator complex [GO:0090575] Also known as: SMAD1-SMAD4 protein complex, SMAD2-SMAD3-SMAD4 protein complex, SMAD2-SMAD4 protein complex, SMAD3-SMAD4 protein complex